{
  "gene_name": "Solute carrier organic anion transporter family member 1B3",
  "gene": "UniProtKB:Q9NPD5",
  "term_label": "bile acid transmembrane transporter activity",
  "term_id": "GO:0015125",
  "gene_symbol": "SLCO1B3"
}